regulation of apolipoprotein A-I-mediated signaling pathway [GO:1905094] (biological process) Subtypes: negative regulation of apolipoprotein A-I-mediated signaling pathway [GO:1905095], GO:1905096 References: PMID:25084135 Sources: GOC:BHF, GOC:BHF_miRNA, GOC:TermGenie, GOC:bc, GO_REF:0000058 Definition: Any process that modulates the frequency, rate or extent of apolipoprotein A-I-mediated signaling pathway. Also known as: regulation of apolipoprotein A-I-mediated signalling pathway Relationships: is a type of regulation of signal transduction [GO:0009966]; RO_0002211 apolipoprotein A-I-mediated signaling pathway [GO:0038027]